{
  "gene_name": "Golgin subfamily A member 4",
  "gene_symbol": "GOLGA4",
  "term_label": "Golgi vesicle transport",
  "term_id": "GO:0048193",
  "gene": "UniProtKB:Q13439"
}